{
  "gene": "UniProtKB:Q8TDX6",
  "gene_name": "Chondroitin sulfate N-acetylgalactosaminyltransferase 1",
  "gene_symbol": "CSGALNACT1",
  "term_id": "UNKNOWN:0003",
  "term_label": "Unknown cellular component"
}